oocyte construction [GO:0007308] (biological process) Also known as: oocyte arrangement Definition: The synthesis, deposition, and organization of the materials in a cell of an ovary; where the cell can then undergo meiosis and form an ovum. An example of this is found in Drosophila melanogaster. Relationships: is a type of developmental process involved in reproduction [GO:0003006]; is a type of GO:0048469; is part of oocyte development [GO:0048599] Sources: GOC:dph, GOC:ems, GOC:mtg_sensu, GOC:tb, ISBN:0198506732